triglyceride metabolic process [GO:0006641] (biological process) Definition: The chemical reactions and pathways involving triglyceride, any triester of glycerol. The three fatty acid residues may all be the same or differ in any permutation. Triglycerides are important components of plant oils, animal fats and animal plasma lipoproteins. Also known as: triacylglycerol metabolic process, triacylglycerol metabolism, triglyceride metabolism Regulation: regulated by regulation of triglyceride metabolic process [GO:0090207]; positively regulated by positive regulation of triglyceride metabolic process [GO:0090208]; negatively regulated by negative regulation of triglyceride metabolic process [GO:0090209] Relationships: is a type of acylglycerol metabolic process [GO:0006639] Subtypes: triglyceride mobilization [GO:0006642], triglyceride biosynthetic process [GO:0019432], triglyceride catabolic process [GO:0019433], triglyceride acyl-chain remodeling [GO:0036153] Sources: ISBN:0198506732